{
  "gene": "UniProtKB:Q8TBF4",
  "term_id": "UNKNOWN:0001",
  "gene_name": "Zinc finger CCHC-type and RNA-binding motif-containing protein 1",
  "gene_symbol": "ZCRB1",
  "term_label": "Unknown molecular function"
}